polyphosphate import into vacuole [GO:0180042] (biological process) Definition: The directed movement of polyphosphate into the vacuole across the vacuolar membrane. References: PMID:37066886 Relationships: is a type of inorganic anion transport [GO:0015698]; is a type of vacuolar transmembrane transport [GO:0034486]